{
  "gene_name": "Sorting nexin-4",
  "gene_symbol": "SNX4",
  "term_id": "GO:2000786",
  "term_label": "positive regulation of autophagosome assembly",
  "gene": "UniProtKB:O95219"
}